{
  "term_label": "plasma membrane",
  "gene": "UniProtKB:P30874",
  "term_id": "GO:0005886",
  "gene_symbol": "SSTR2",
  "gene_name": "Somatostatin receptor type 2"
}